{
  "term_label": "hydrolase activity, acting on carbon-nitrogen (but not peptide) bonds",
  "gene_symbol": "NAAA",
  "term_id": "GO:0016810",
  "gene": "UniProtKB:Q02083",
  "gene_name": "N-acylethanolamine-hydrolyzing acid amidase"
}